{
  "term_id": "GO:0045121",
  "gene": "UniProtKB:Q96QB1",
  "gene_name": "Rho GTPase-activating protein 7",
  "term_label": "membrane raft",
  "gene_symbol": "DLC1"
}